{
  "gene_name": "Metallothionein-1G",
  "gene_symbol": "MT1G",
  "term_label": "metal ion binding",
  "term_id": "GO:0046872",
  "gene": "UniProtKB:P13640"
}